{
  "gene": "UniProtKB:Q6ZN57",
  "gene_name": "Zinc finger protein ZFP2",
  "term_id": "GO:0006357",
  "gene_symbol": "ZFP2",
  "term_label": "regulation of transcription by RNA polymerase II"
}